{
  "term_id": "GO:0006281",
  "gene_name": "DNA topoisomerase 3-beta-1",
  "gene": "UniProtKB:O95985",
  "gene_symbol": "TOP3B",
  "term_label": "DNA repair"
}